{
  "gene_symbol": "CRYAB",
  "gene": "UniProtKB:P02511",
  "term_id": "GO:0051082",
  "gene_name": "Alpha-crystallin B chain",
  "term_label": "unfolded protein binding"
}